{
  "term_id": "GO:0000711",
  "gene_name": "Synaptonemal complex protein 1",
  "gene": "UniProtKB:Q15431",
  "term_label": "meiotic DNA repair synthesis",
  "gene_symbol": "SYCP1"
}